specification of mesonephric connecting tubule identity [GO:0061281] (biological process) Also known as: specification of mesonephric collecting tubule identity Relationships: is a type of specification of mesonephric nephron tubule identity [GO:0061282]; is_a specification of connecting tubule identity [GO:0072085]; is part of mesonephric connecting tubule development [GO:0061272] Sources: GOC:mtg_kidney_jan10 Definition: The process in which the connecting tubule of the mesonephric nephron acquires its identity.